negative regulation of adenylate cyclase-inhibiting dopamine receptor signaling pathway [GO:1904991] (biological process) References: PMID:26554819 Sources: GOC:TermGenie, GOC:kmv, GO_REF:0000058 Also known as: down regulation of adenylate cyclase-inhibiting dopamine receptor signaling pathway, down regulation of dopamine receptor, adenylate cyclase inhibiting pathway, down regulation of dopamine receptor, adenylyl cyclase inhibiting pathway, down regulation of inhibition of adenylate cyclase activity by dopamine receptor signalling pathway, down-regulation of adenylate cyclase-inhibiting dopamine receptor signaling pathway, down-regulation of dopamine receptor, adenylate cyclase inhibiting pathway, down-regulation of dopamine receptor, adenylyl cyclase inhibiting pathway, down-regulation of inhibition of adenylate cyclase activity by dopamine receptor signalling pathway, downregulation of adenylate cyclase-inhibiting dopamine receptor signaling pathway, downregulation of dopamine receptor, adenylate cyclase inhibiting pathway, downregulation of dopamine receptor, adenylyl cyclase inhibiting pathway, downregulation of inhibition of adenylate cyclase activity by dopamine receptor signalling pathway, negative regulation of dopamine receptor, adenylate cyclase inhibiting pathway, negative regulation of dopamine receptor, adenylyl cyclase inhibiting pathway, negative regulation of inhibition of adenylate cyclase activity by dopamine receptor signalling pathway, inhibition of adenylate cyclase-inhibiting dopamine receptor signaling pathway, inhibition of dopamine receptor, adenylate cyclase inhibiting pathway, inhibition of dopamine receptor, adenylyl cyclase inhibiting pathway, inhibition of inhibition of adenylate cyclase activity by dopamine receptor signalling pathway, down regulation of inhibition of adenylate cyclase activity by dopamine receptor signaling pathway, down-regulation of inhibition of adenylate cyclase activity by dopamine receptor signaling pathway, downregulation of inhibition of adenylate cyclase activity by dopamine receptor signaling pathway, inhibition of inhibition of adenylate cyclase activity by dopamine receptor signaling pathway, negative regulation of inhibition of adenylate cyclase activity by dopamine receptor signaling pathway Definition: Any process that stops, prevents or reduces the frequency, rate or extent of adenylate cyclase-inhibiting dopamine receptor signaling pathway. Relationships: is a type of negative regulation of dopamine receptor signaling pathway [GO:0060160]; is a type of regulation of adenylate cyclase-inhibiting dopamine receptor signaling pathway [GO:1904990]; negatively regulates adenylate cyclase-inhibiting dopamine receptor signaling pathway [GO:0007195]